acrosin binding [GO:0032190] (molecular function) Also known as: acrosin heavy chain binding, acrosin light chain binding References: PMID:12398221 Sources: GOC:mah Definition: Binding to acrosin, a protein that is found in the acrosomes of sperm and possesses protease and carbohydrate binding activities. Relationships: is a type of enzyme binding [GO:0019899]